{
  "gene": "UniProtKB:Q8WZ74",
  "term_label": "Unknown molecular function",
  "gene_symbol": "CTTNBP2",
  "term_id": "UNKNOWN:0001",
  "gene_name": "Cortactin-binding protein 2"
}